{
  "gene": "UniProtKB:Q8NHW5",
  "gene_symbol": "RPLP0P6",
  "term_label": "large ribosomal subunit rRNA binding",
  "term_id": "GO:0070180",
  "gene_name": "Putative ribosomal protein uL10-like"
}